{
  "gene_name": "Protein ABHD11",
  "term_label": "lipid metabolic process",
  "gene": "UniProtKB:Q8NFV4",
  "term_id": "GO:0006629",
  "gene_symbol": "ABHD11"
}